swim bladder development [GO:0048794] (biological process) Relationships: is a type of GO:0048513 Sources: GOC:mh Definition: The process whose specific outcome is the progression of the swim bladder over time, from its formation to the mature structure. The swim bladder is used by some fishes to maintain buoyancy and may function in addition as a sound producing organ, a sound receptor, and a respiratory organ. Also known as: gas bladder development